{
  "gene_symbol": "BNIP5",
  "term_id": "UNKNOWN:0001",
  "term_label": "Unknown molecular function",
  "gene_name": "Protein BNIP5",
  "gene": "UniProtKB:P0C671"
}